endocardial endothelium development [GO:0061147] (biological process) Definition: The progression of the endocardial endothelium over time, from its initial formation to the mature structure. The endocardium is an anatomical structure comprised of an endothelium and an extracellular matrix that forms the innermost layer of tissue of the heart, and lines the heart chambers. Relationships: is a type of endothelium development [GO:0003158]; is part of endocardium development [GO:0003157] Sources: GOC:dph